{
  "term_label": "cyclic-GMP-AMP transmembrane import across plasma membrane",
  "gene_name": "Leucine-rich repeat protein SHOC-2",
  "term_id": "GO:0140361",
  "gene_symbol": "SHOC2",
  "gene": "UniProtKB:Q9UQ13"
}